{
  "term_id": "GO:0007018",
  "gene": "UniProtKB:O75037",
  "term_label": "microtubule-based movement",
  "gene_symbol": "KIF21B",
  "gene_name": "Kinesin-like protein KIF21B"
}